regulation of lymphocyte migration [GO:2000401] (biological process) Sources: GOC:mah Definition: Any process that modulates the frequency, rate or extent of lymphocyte migration. Relationships: is a type of regulation of mononuclear cell migration [GO:0071675]; regulates lymphocyte migration [GO:0072676] Subtypes: regulation of lymphocyte chemotaxis [GO:1901623], GO:2000402, positive regulation of lymphocyte migration [GO:2000403], regulation of T cell migration [GO:2000404]